rhamnogalacturonan endolyase activity [GO:0102210] (molecular function) Definition: Catalysis of the reaction: H2O + a rhamnogalacturonan type I = [rhamnogalacturonan I oligosaccharide]-alpha-L-rhamnose + 4-deoxy-4,5-unsaturated D-galactopyranosyluronate-[rhamnogalacturonan I oligosaccharide]. Relationships: is a type of carbon-oxygen lyase activity, acting on polysaccharides [GO:0016837] Sources: EC:4.2.2.23, GOC:pz